{
  "gene": "UniProtKB:A8MYP8",
  "term_id": "UNKNOWN:0001",
  "gene_name": "Outer dense fiber protein 3B",
  "gene_symbol": "CIMAP1B",
  "term_label": "Unknown molecular function"
}